{
  "gene_symbol": "ECH1",
  "gene_name": "Delta(3,5)-Delta(2,4)-dienoyl-CoA isomerase, mitochondrial",
  "term_label": "Unknown biological process",
  "term_id": "UNKNOWN:0002",
  "gene": "UniProtKB:Q13011"
}